{
  "gene_name": "Pre-B-cell leukemia transcription factor 2",
  "term_label": "eye development",
  "term_id": "GO:0001654",
  "gene_symbol": "PBX2",
  "gene": "UniProtKB:P40425"
}